{
  "gene": "UniProtKB:Q07157",
  "term_id": "GO:0050839",
  "gene_name": "Tight junction protein ZO-1",
  "gene_symbol": "TJP1",
  "term_label": "cell adhesion molecule binding"
}